{
  "gene_name": "Receptor-type tyrosine-protein phosphatase N2",
  "gene": "UniProtKB:Q92932",
  "term_label": "insulin secretion involved in cellular response to glucose stimulus",
  "term_id": "GO:0035773",
  "gene_symbol": "PTPRN2"
}